spermidine metabolic process [GO:0008216] (biological process) Also known as: spermidine metabolism Sources: GOC:ai Relationships: is a type of polyamine metabolic process [GO:0006595] Definition: The chemical reactions and pathways involving spermidine, N-(3-aminopropyl)-1,4-diaminobutane. Subtypes: GO:0008295, spermidine acetylation [GO:0032918], spermidine catabolic process [GO:0046203], spermidine deacetylation [GO:0106048]